{
  "gene_symbol": "CXorf65",
  "term_id": "UNKNOWN:0001",
  "gene": "UniProtKB:A6NEN9",
  "gene_name": "Uncharacterized protein CXorf65",
  "term_label": "Unknown molecular function"
}